{
  "gene_name": "Disintegrin and metalloproteinase domain-containing protein 8",
  "gene_symbol": "ADAM8",
  "term_label": "regulation of cell-cell adhesion",
  "gene": "UniProtKB:P78325",
  "term_id": "GO:0022407"
}